{
  "gene": "UniProtKB:Q96CN7",
  "term_id": "UNKNOWN:0001",
  "gene_name": "Isochorismatase domain-containing protein 1",
  "gene_symbol": "ISOC1",
  "term_label": "Unknown molecular function"
}